regulation of chronic inflammatory response [GO:0002676] (biological process) Definition: Any process that modulates the frequency, rate, or extent of a chronic inflammatory response. Sources: GOC:add Subtypes: regulation of granuloma formation [GO:0002631], negative regulation of chronic inflammatory response [GO:0002677], positive regulation of chronic inflammatory response [GO:0002678], regulation of chronic inflammatory response to antigenic stimulus [GO:0002874], GO:0002880 Relationships: is a type of regulation of inflammatory response [GO:0050727]; regulates GO:0002544